CP2 mannose-ethanolamine phosphotransferase activity [GO:0051267] (molecular function) Also known as: CP2 EtN-P transferase activity, CP2 ethanolamine phosphate transferase activity, CP2 phosphoethanolamine transferase activity, addition of ethanolamine phosphate to mannose of GPI precursor CP2, gpi7 activity Relationships: is a type of GO:0051377 References: PMID:14985347, PMID:15452134 Definition: Catalysis of the reaction: ethanolamine phosphate + Man-alpha-(1,2)-Man-alpha-(1,2)-Man-alpha-(1,6)-R = Man-alpha-(1,2)-Man-alpha-6-P-EtN-(1,2)-Man-alpha-(1,6)-R; R is Man-alpha(1,4)-GlcNH2-inositol-phosphate-lipid. This reaction is the transfer of ethanolamine phosphate to C6 of second mannose in the GPI lipid precursor CP2.